{
  "gene_name": "Interferon alpha-7",
  "gene_symbol": "IFNA7",
  "gene": "UniProtKB:P01567",
  "term_id": "GO:0002286",
  "term_label": "T cell activation involved in immune response"
}